{
  "term_label": "Unknown biological process",
  "gene": "UniProtKB:O60869",
  "term_id": "UNKNOWN:0002",
  "gene_symbol": "EDF1",
  "gene_name": "Endothelial differentiation-related factor 1"
}